phosphoenolpyruvate transport [GO:0015714] (biological process) Subtypes: GO:0089722 Sources: GOC:krc Relationships: is a type of monocarboxylic acid transport [GO:0015718]; is a type of organophosphate ester transport [GO:0015748] Definition: The directed movement of phosphoenolpyruvate into, out of or within a cell, or between cells, by means of some agent such as a transporter or pore.